{
  "gene_symbol": "C17orf113",
  "gene_name": "Uncharacterized protein C17orf113",
  "gene": "UniProtKB:A0A1B0GUU1",
  "term_label": "Unknown biological process",
  "term_id": "UNKNOWN:0002"
}